{
  "gene_name": "Mitogen-activated protein kinase 12",
  "term_id": "GO:0005737",
  "term_label": "cytoplasm",
  "gene": "UniProtKB:P53778",
  "gene_symbol": "MAPK12"
}